{
  "term_label": "Unknown biological process",
  "gene_symbol": "UMAD1",
  "gene": "UniProtKB:C9J7I0",
  "term_id": "UNKNOWN:0002",
  "gene_name": "UBAP1-MVB12-associated (UMA)-domain containing protein 1"
}